{
  "term_id": "UNKNOWN:0003",
  "gene_symbol": "TRBJ1-2",
  "gene": "UniProtKB:A0A0J9YX06",
  "gene_name": "T cell receptor beta joining 1-2",
  "term_label": "Unknown cellular component"
}